{
  "term_id": "UNKNOWN:0001",
  "gene_symbol": "RBAKDN",
  "term_label": "Unknown molecular function",
  "gene": "UniProtKB:A6NC62",
  "gene_name": "Putative RBAK downstream neighbor protein"
}